{
  "gene_name": "2',3'-cyclic-nucleotide 3'-phosphodiesterase",
  "term_id": "UNKNOWN:0002",
  "term_label": "Unknown biological process",
  "gene": "UniProtKB:P09543",
  "gene_symbol": "CNP"
}